glutathione binding [GO:0043295] (molecular function) Sources: GOC:bf, ISBN:0198506732 Relationships: is a type of anion binding [GO:0043168]; is a type of modified amino acid binding [GO:0072341]; is a type of oligopeptide binding [GO:1900750]; is a type of sulfur compound binding [GO:1901681] Definition: Binding to glutathione; a tripeptide composed of the three amino acids cysteine, glutamic acid and glycine.